lymphotoxin A production [GO:0032641] (biological process) Regulation: regulated by regulation of lymphotoxin A production [GO:0032681]; negatively regulated by negative regulation of lymphotoxin A production [GO:0032721]; positively regulated by GO:0032761 Relationships: is a type of GO:0019538; is a type of tumor necrosis factor superfamily cytokine production [GO:0071706] Also known as: LTA production, TNF-B production, TNF-beta production, lymphotoxin-alpha production, tumor necrosis factor-beta production, lymphotoxin A biosynthetic process, lymphotoxin A synthesis, lymphotoxin A formation Note: Note that this term is in the subset of terms that should not be used for direct gene product annotation. Instead, select one of the 'regulation' children terms. Sources: GOC:jl Definition: The chemical reactions and pathways resulting in the formation of the cytokine lymphotoxin A.